sepal structural organization [GO:0048454] (biological process) Relationships: is a type of floral organ structural organization [GO:0048450]; is part of sepal morphogenesis [GO:0048447] Sources: GOC:jid Also known as: sepal structural organisation Definition: The process that contributes to the act of creating the structural organization of the sepal. This process pertains to the physical shaping of a rudimentary structure.